2-chloro-4-carboxymethylenebut-2-en-1,4-olide isomerase activity [GO:0047466] (molecular function) Relationships: is_a cis-trans isomerase activity [GO:0016859] Sources: EC:5.2.1.10, RHEA:10924 Also known as: 2-chloro-4-carboxymethylenebut-2-en-1,4-olide cis-trans-isomerase activity, 2-chlorocarboxymethylenebutenolide isomerase activity, chlorodienelactone isomerase activity Definition: Catalysis of the reaction: cis-2-chloro-4-carboxymethylenebut-2-en-1,4-olide = trans-2-chloro-4-carboxymethylenebut-2-en-1,4-olide.